{
  "gene_name": "Tubby-related protein 4",
  "gene_symbol": "TULP4",
  "gene": "UniProtKB:Q9NRJ4",
  "term_id": "UNKNOWN:0003",
  "term_label": "Unknown cellular component"
}